acetylalkylglycerol acetylhydrolase activity [GO:0047378] (molecular function) Relationships: is a type of GO:0052689 Sources: EC:3.1.1.71, RHEA:11552 Also known as: 2-acetyl-1-alkyl-sn-glycerol acetylhydrolase activity, alkylacetylglycerol acetylhydrolase activity Definition: Catalysis of the reaction: 2-acetyl-1-alkyl-sn-glycerol + H2O = 1-alkyl-sn-glycerol + acetate + H+.